{
  "gene": "UniProtKB:Q01196",
  "term_label": "chondrocyte differentiation",
  "gene_name": "Runt-related transcription factor 1",
  "term_id": "GO:0002062",
  "gene_symbol": "RUNX1"
}